{
  "term_label": "Unknown biological process",
  "term_id": "UNKNOWN:0002",
  "gene": "UniProtKB:A0A1B0GVN3",
  "gene_name": "Uncharacterized protein C2orf92",
  "gene_symbol": "C2orf92"
}